negative regulation of intracellular estrogen receptor signaling pathway [GO:0033147] (BP) Definition: Any process that stops, prevents, or reduces the frequency, rate or extent of the activity of an intracellular estrogen receptor signaling pathway. Sources: GOC:mah Relationships: is_a negative regulation of intracellular steroid hormone receptor signaling pathway [GO:0033144]; is a type of GO:0033146; negatively regulates GO:0030520 Also known as: negative regulation of estrogen receptor signaling pathway, negative regulation of estrogen receptor signalling pathway